alpha-tocopherol omega-hydroxylase activity [GO:0052871] (molecular function) Relationships: is a type of oxidoreductase activity, acting on paired donors, with incorporation or reduction of molecular oxygen, reduced flavin or flavoprotein as one donor, and incorporation of one atom of oxygen [GO:0016712] Definition: Catalysis of the reaction: (+)-alpha-tocopherol + O2 + reduced [NADPH--hemoprotein reductase] = 13-hydroxy-alpha-tocopherol + H+ + H2O + oxidized [NADPH--hemoprotein reductase]. Sources: RHEA:45108 Also known as: alpha-tocopherol 13-hydroxylase activity